chloroplast nucleoid [GO:0042644] (CC) Definition: The region of a chloroplast to which the DNA is confined. Sources: GOC:jl Relationships: is a type of plastid nucleoid [GO:0042646]; is part of chloroplast stroma [GO:0009570]